dorsal cochlear nucleus development [GO:0021748] (biological process) Sources: GOC:cls, GOC:curators, GOC:dgh, GOC:dph, GOC:jid Relationships: is a type of GO:0021747 Definition: The process whose specific outcome is the progression of the dorsal cochlear nucleus over time, from its formation to the mature structure.